seed trichome elongation [GO:0090378] (biological process) Sources: GOC:tb Definition: The process in which a seed trichome irreversibly increases in size in one [spatial] dimension or along one axis, resulting in the morphogenesis of the cell. Note: The increase in length of the seed trichome without cell division. Elongation is defined to be from 5 to 20 DPA in Gossypium spp. Relationships: is a type of GO:0003006; is a type of unidimensional cell growth [GO:0009826]; is a type of GO:0022412; is part of seed trichome differentiation [GO:0090376]